{
  "gene_symbol": "ANAPC15",
  "term_id": "GO:0090266",
  "term_label": "regulation of mitotic cell cycle spindle assembly checkpoint",
  "gene": "UniProtKB:P60006",
  "gene_name": "Anaphase-promoting complex subunit 15"
}